nitric oxide metabolic process [GO:0046209] (biological process) Also known as: nitric oxide metabolism Subtypes: GO:0006809, GO:0046210 Definition: The chemical reactions and pathways involving nitric oxide, nitrogen monoxide (NO), a colorless gas only slightly soluble in water. Sources: GOC:ai Regulation: regulated by regulation of nitric oxide metabolic process [GO:0080164] Relationships: is a type of reactive nitrogen species metabolic process [GO:2001057]